{
  "term_id": "GO:0005739",
  "gene_name": "Small ribosomal subunit protein mS38",
  "term_label": "mitochondrion",
  "gene": "UniProtKB:Q9NWT8",
  "gene_symbol": "AURKAIP1"
}